{
  "gene_symbol": "ANTXR1",
  "gene": "UniProtKB:Q9H6X2",
  "gene_name": "Anthrax toxin receptor 1",
  "term_label": "cell surface",
  "term_id": "GO:0009986"
}